{
  "gene_symbol": "CELF1",
  "term_id": "GO:0005737",
  "gene_name": "CUGBP Elav-like family member 1",
  "term_label": "cytoplasm",
  "gene": "UniProtKB:Q92879"
}